{
  "gene": "UniProtKB:P0DML2",
  "gene_name": "Chorionic somatomammotropin hormone 1",
  "term_id": "GO:0048513",
  "gene_symbol": "CSH1",
  "term_label": "animal organ development"
}